{
  "gene": "UniProtKB:Q9UPT6",
  "term_id": "GO:0005078",
  "gene_symbol": "MAPK8IP3",
  "term_label": "MAP-kinase scaffold activity",
  "gene_name": "C-Jun-amino-terminal kinase-interacting protein 3"
}